{
  "gene_name": "Protein Mpv17",
  "term_label": "channel activity",
  "gene": "UniProtKB:P39210",
  "gene_symbol": "MPV17",
  "term_id": "GO:0015267"
}